{
  "gene": "UniProtKB:Q14678",
  "term_id": "UNKNOWN:0001",
  "term_label": "Unknown molecular function",
  "gene_symbol": "KANK1",
  "gene_name": "KN motif and ankyrin repeat domain-containing protein 1"
}